{
  "term_label": "keratin filament",
  "gene_symbol": "KRT20",
  "term_id": "GO:0045095",
  "gene": "UniProtKB:P35900",
  "gene_name": "Keratin, type I cytoskeletal 20"
}